diestrus [GO:0060207] (biological process) Relationships: is a type of estrous cycle phase [GO:0060206] Definition: The estrous cycle phase which is a period of sexual quiescence and represents the phase of the mature corpus luteum. Note: Note that this term should not be used for direct annotation. If you are trying to make an annotation to x phase, it is likely that the correct annotation is 'regulation of x/y phase transition' or to a process which occurs during the reported phase. To capture the phase when a specific location or process is observed, the phase term can be used in an annotation extension (PMID:24885854) applied to a cellular component term (with the relation exists_during) or a biological process term (with the relation happens_during). Sources: GOC:dph, ISBN:0721662544